{
  "gene": "UniProtKB:Q8NCT1",
  "gene_name": "Arrestin domain-containing protein 4",
  "gene_symbol": "ARRDC4",
  "term_id": "UNKNOWN:0002",
  "term_label": "Unknown biological process"
}